{
  "term_id": "GO:0005737",
  "gene_name": "Ribose-phosphate pyrophosphokinase 1",
  "gene": "UniProtKB:P60891",
  "gene_symbol": "PRPS1",
  "term_label": "cytoplasm"
}